{
  "gene_symbol": "SEMA3E",
  "gene_name": "Semaphorin-3E",
  "gene": "UniProtKB:O15041",
  "term_id": "GO:0050919",
  "term_label": "negative chemotaxis"
}